dark adaptation [GO:1990603] (biological process) Definition: The process by which the rods of the retina gradually become fully responsive to dim light when no longer exposed to bright light. Note: The proteins RGS9-1 and Gb5L localize to the rod inner segment during dark adaptation, but to the rod outer segment during light adaptation. PMID:23555598 Relationships: is a type of cellular response to absence of light [GO:0071485] References: PMID:11420957, PMID:35268448 Sources: GOC:hjd, https://www.ncbi.nlm.nih.gov/books/NBK11525/